{
  "term_label": "mRNA cleavage and polyadenylation specificity factor complex",
  "gene": "UniProtKB:A0A1W2PQ27",
  "term_id": "GO:0005847",
  "gene_name": "RNA polymerase II subunit A C-terminal domain phosphatase SSU72 like protein 1",
  "gene_symbol": "SSU72L1"
}